syringal lignin catabolic process [GO:1901065] (biological process) Sources: GOC:TermGenie, GOC:mengo_curators Also known as: S-lignin catabolic process, syringal lignin breakdown, syringal lignin catabolism, syringal lignin degradation Regulation: regulated by regulation of syringal lignin catabolic process [GO:1901469]; negatively regulated by negative regulation of syringal lignin catabolic process [GO:1901470]; positively regulated by positive regulation of syringal lignin catabolic process [GO:1901471] Relationships: is a type of lignin catabolic process [GO:0046274] Definition: The chemical reactions and pathways resulting in the breakdown of syringal lignin.